chloroplast accumulation movement [GO:0009904] (biological process) References: PMID:11978863 Sources: GOC:tb Definition: The relocation process in which chloroplasts in photosynthetic cells move toward a brighter area in a cell to optimize photosynthesis. Also known as: low-fluence-rate response Relationships: is a type of chloroplast relocation [GO:0009902]